{
  "gene_symbol": "TRMT6",
  "gene": "UniProtKB:Q9UJA5",
  "gene_name": "tRNA (adenine(58)-N(1))-methyltransferase non-catalytic subunit TRM6",
  "term_label": "nucleus",
  "term_id": "GO:0005634"
}